{
  "gene_name": "Voltage-dependent T-type calcium channel subunit alpha-1H",
  "term_id": "GO:0005891",
  "gene": "UniProtKB:O95180",
  "gene_symbol": "CACNA1H",
  "term_label": "voltage-gated calcium channel complex"
}